{
  "gene_symbol": "TLR2",
  "gene": "UniProtKB:O60603",
  "gene_name": "Toll-like receptor 2",
  "term_id": "GO:0005886",
  "term_label": "plasma membrane"
}